{
  "term_id": "GO:0005911",
  "gene_symbol": "IGSF11",
  "gene": "UniProtKB:Q5DX21",
  "term_label": "cell-cell junction",
  "gene_name": "Immunoglobulin superfamily member 11"
}